{
  "gene_symbol": "HOXC12",
  "gene": "UniProtKB:P31275",
  "term_id": "GO:1990837",
  "term_label": "sequence-specific double-stranded DNA binding",
  "gene_name": "Homeobox protein Hox-C12"
}